{
  "gene": "UniProtKB:Q32M78",
  "term_label": "nucleus",
  "gene_symbol": "ZNF699",
  "term_id": "GO:0005634",
  "gene_name": "Zinc finger protein 699"
}